ATP metabolic process [GO:0046034] (biological process) Regulation: regulated by GO:1903578; negatively regulated by negative regulation of ATP metabolic process [GO:1903579]; positively regulated by positive regulation of ATP metabolic process [GO:1903580] Sources: GOC:go_curators Relationships: is a type of purine ribonucleotide metabolic process [GO:0009150]; is_a purine ribonucleoside triphosphate metabolic process [GO:0009205] Subtypes: glycolytic process [GO:0006096], ATP biosynthetic process [GO:0006754], sulphoglycolysis [GO:0061722], GO:1990966 Also known as: ATP metabolism Definition: The chemical reactions and pathways involving ATP, adenosine triphosphate, a universally important coenzyme and enzyme regulator.